{
  "gene_symbol": "CCL21",
  "term_label": "chemokine activity",
  "term_id": "GO:0008009",
  "gene_name": "C-C motif chemokine 21",
  "gene": "UniProtKB:O00585"
}